{
  "term_id": "GO:0005739",
  "term_label": "mitochondrion",
  "gene_symbol": "ABCB10",
  "gene": "UniProtKB:Q9NRK6",
  "gene_name": "ATP-binding cassette sub-family B member 10, mitochondrial"
}